{
  "gene_symbol": "ADAMTS2",
  "term_id": "GO:0004222",
  "term_label": "metalloendopeptidase activity",
  "gene": "UniProtKB:O95450",
  "gene_name": "A disintegrin and metalloproteinase with thrombospondin motifs 2"
}